{
  "gene_name": "Sushi, von Willebrand factor type A, EGF and pentraxin domain-containing protein 1",
  "term_label": "epidermis development",
  "gene": "UniProtKB:Q4LDE5",
  "term_id": "GO:0008544",
  "gene_symbol": "SVEP1"
}